{
  "gene_symbol": "CAAP1",
  "gene": "UniProtKB:Q9H8G2",
  "term_label": "Unknown molecular function",
  "term_id": "UNKNOWN:0001",
  "gene_name": "Caspase activity and apoptosis inhibitor 1"
}